{
  "gene_symbol": "CACTIN",
  "gene": "UniProtKB:Q8WUQ7",
  "gene_name": "Splicing factor Cactin",
  "term_label": "mRNA cis splicing, via spliceosome",
  "term_id": "GO:0045292"
}